{
  "gene": "UniProtKB:P62913",
  "gene_name": "Large ribosomal subunit protein uL5",
  "term_id": "GO:0006412",
  "term_label": "translation",
  "gene_symbol": "RPL11"
}